positive regulation of ephrin receptor signaling pathway [GO:1901189] (biological process) Sources: GOC:BHF, GOC:TermGenie Relationships: is a type of positive regulation of signal transduction [GO:0009967]; is a type of regulation of ephrin receptor signaling pathway [GO:1901187]; positively regulates ephrin receptor signaling pathway [GO:0048013] Definition: Any process that activates or increases the frequency, rate or extent of ephrin receptor signaling pathway. Also known as: activation of Eph receptor signaling pathway, activation of Eph receptor signalling pathway, positive regulation of Eph receptor signaling pathway, positive regulation of Eph receptor signalling pathway, up regulation of Eph receptor signaling pathway, up regulation of Eph receptor signalling pathway, up regulation of ephrin receptor signaling pathway, up-regulation of Eph receptor signaling pathway, up-regulation of Eph receptor signalling pathway, up-regulation of ephrin receptor signaling pathway, upregulation of Eph receptor signaling pathway, upregulation of Eph receptor signalling pathway, upregulation of ephrin receptor signaling pathway, activation of ephrin receptor signaling pathway